negative regulation of neutrophil differentiation [GO:0045659] (biological process) Relationships: is_a negative regulation of granulocyte differentiation [GO:0030853]; is a type of regulation of neutrophil differentiation [GO:0045658]; negatively regulates neutrophil differentiation [GO:0030223] Also known as: down regulation of neutrophil differentiation, down-regulation of neutrophil differentiation, downregulation of neutrophil differentiation, inhibition of neutrophil differentiation Definition: Any process that stops, prevents, or reduces the frequency, rate or extent of neutrophil differentiation. Sources: GOC:go_curators